{
  "gene_name": "Acetyl-CoA acetyltransferase, mitochondrial",
  "gene_symbol": "ACAT1",
  "gene": "UniProtKB:P24752",
  "term_id": "UNKNOWN:0002",
  "term_label": "Unknown biological process"
}